{
  "gene_name": "Band 4.1-like protein 4B",
  "gene_symbol": "EPB41L4B",
  "gene": "UniProtKB:Q9H329",
  "term_id": "GO:0005856",
  "term_label": "cytoskeleton"
}